{
  "gene": "UniProtKB:Q6P988",
  "gene_name": "Palmitoleoyl-protein carboxylesterase NOTUM",
  "term_label": "negative regulation of canonical Wnt signaling pathway",
  "gene_symbol": "NOTUM",
  "term_id": "GO:0090090"
}